{
  "gene_symbol": "RNF135",
  "term_label": "regulation of innate immune response",
  "gene": "UniProtKB:Q8IUD6",
  "gene_name": "E3 ubiquitin-protein ligase RNF135",
  "term_id": "GO:0045088"
}